C-terminal protein demethylation [GO:1990577] (biological process) References: PMID:11060018 Relationships: is a type of protein demethylation [GO:0006482] Definition: The removal of a methyl group from the C-terminal amino acid of a protein.